{
  "gene": "UniProtKB:P10398",
  "gene_symbol": "ARAF",
  "gene_name": "Serine_threonine-protein kinase A-Raf",
  "term_label": "cytosol",
  "term_id": "GO:0005829"
}